detection of glucocorticoid hormone stimulus [GO:0051468] (BP) Sources: GOC:ai Relationships: is_a response to glucocorticoid [GO:0051384]; is_a detection of steroid hormone stimulus [GO:0051467] Definition: The series of events by which a glucocorticoid hormone stimulus is received by a cell and converted into a molecular signal. Glucocorticoids are hormonal C21 corticosteroids synthesized from cholesterol with the ability to bind with the cortisol receptor and trigger similar effects. Glucocorticoids act primarily on carbohydrate and protein metabolism, and have anti-inflammatory effects.